protein-containing complex localization to centriolar satellite [GO:0140706] (biological process) Relationships: is a type of protein-containing complex localization [GO:0031503] Definition: A protein-containing complex localization by which the complex is transported to, or maintained in, the centriolar satellite. References: PMID:27979967